mesonephric glomerular parietal epithelial cell fate commitment [GO:0061255] (biological process) Definition: The process in which the developmental fate of a cell becomes restricted such that it will develop into a mesonephric glomerular parietal epithelial cell. Mesonephric glomerular parietal epithelial cells are specialized epithelial cells that form tight junctions as a barrier to protein transport. These cells may also give rise to podocytes. Sources: GOC:mtg_kidney_jan10 Relationships: is a type of mesonephric glomerular epithelial cell fate commitment [GO:0061252]; is a type of glomerular parietal epithelial cell fate commitment [GO:0072147]; is part of mesonephric glomerular parietal epithelial cell differentiation [GO:0061253]